MPP7-DLG1-LIN7 complex [GO:0097025] (cellular component) References: PMID:17237226 Sources: GOC:BHF Definition: A heterotrimeric protein complex formed by the association of MMP7, DLG1 and either LIN7A or LIN7C; regulates the stability and localization of DLG1 to cell junctions. Relationships: is a type of plasma membrane protein complex [GO:0098797]; is part of adherens junction [GO:0005912]